{
  "gene": "UniProtKB:O60381",
  "term_label": "DNA-binding transcription factor activity, RNA polymerase II-specific",
  "gene_name": "HMG box-containing protein 1",
  "term_id": "GO:0000981",
  "gene_symbol": "HBP1"
}